adaxial/abaxial pattern specification [GO:0009955] (biological process) Sources: GOC:dph, GOC:isa_complete, GOC:tb Also known as: adaxial/abaxial pattern formation Relationships: is a type of regionalization [GO:0003002] Definition: The regionalization process in which differences in cell differentiation along the adaxial/abaxial are generated. Adaxial refers to being situated toward an axis of an anatomical structure. Abaxial refers to being situated away from an axis of an anatomical structure. Regulation: regulated by regulation of adaxial/abaxial pattern formation [GO:2000011]